{
  "term_id": "GO:0051015",
  "term_label": "actin filament binding",
  "gene_symbol": "AIF1",
  "gene_name": "Allograft inflammatory factor 1",
  "gene": "UniProtKB:P55008"
}